{
  "term_id": "UNKNOWN:0001",
  "gene": "UniProtKB:O00273",
  "gene_name": "DNA fragmentation factor subunit alpha",
  "term_label": "Unknown molecular function",
  "gene_symbol": "DFFA"
}